{
  "term_id": "GO:0097602",
  "gene": "UniProtKB:Q9NXV2",
  "gene_symbol": "KCTD5",
  "gene_name": "BTB_POZ domain-containing protein KCTD5",
  "term_label": "cullin family protein binding"
}